{
  "term_label": "iron-sulfur cluster assembly",
  "gene": "UniProtKB:Q9HD34",
  "gene_name": "LYR motif-containing protein 4",
  "term_id": "GO:0016226",
  "gene_symbol": "LYRM4"
}